HICS complex [GO:0044697] (CC) Relationships: is a type of protein-containing complex [GO:0032991] Definition: A multisubunit complex involved in cytokinesis. In the yeast Saccharomyces cerevisiae this complex consists of Sho1p, Hof1p, Inn1p and Cyk3p proteins. References: PMID:22623719